cell surface receptor signaling pathway via STAT [GO:0097696] (BP) Also known as: STAT signalling pathway, kinase activated-STAT cascade, kinase-STAT cascade, receptor signaling pathway via STAT References: PMID:21534947, PMID:24587195 Sources: GOC:rjd Note: In most species, STAT proteins are activated by members of the JAK (Janus Activated Kinase) family of tyrosine kinases; the term GO:0007259 'JAK-STAT cascade' describes this specificity. In other cases, such as D. discoideum, no JAK orthologs are known, and STAT proteins are activated by tyrosine kinase-like proteins. Subtypes: cell surface receptor signaling pathway via JAK-STAT [GO:0007259] Regulation: regulated by regulation of receptor signaling pathway via STAT [GO:1904892]; RO_0002212 by negative regulation of receptor signaling pathway via STAT [GO:1904893]; RO_0002213 by positive regulation of receptor signaling pathway via STAT [GO:1904894] Relationships: is a type of cell surface receptor signaling pathway [GO:0007166] Definition: An intracellular signal transduction process in which STAT proteins (Signal Transducers and Activators of Transcription) convey a signal to trigger a change in the activity or state of a cell. The STAT cascade begins with receptor activation followed by activation of STAT proteins by kinases. It proceeds through STA dimerization and subsequent nuclear translocation of STAT proteins, and ends with regulation of target gene expression by STAT proteins.